phospholipase C-activating adrenergic receptor signaling pathway [GO:0071882] (BP) Sources: GOC:BHF, GOC:mah, GOC:signaling Also known as: activation of phospholipase C activity by adrenergic receptor signaling pathway, activation of phospholipase C activity by adrenergic receptor signalling pathway, adrenergic receptor, phospholipase C activating pathway Definition: A phospholipase C-activating receptor G protein-coupled receptor signaling pathway initiated by ligand binding to an adrenergic receptor on the surface of a target cell, and ending with the regulation of a downstream cellular process, e.g. transcription. Relationships: is a type of phospholipase C-activating G protein-coupled receptor signaling pathway [GO:0007200]; is a type of GO:0071875